{
  "term_id": "GO:0000981",
  "gene": "UniProtKB:A6NLW8",
  "term_label": "DNA-binding transcription factor activity, RNA polymerase II-specific",
  "gene_name": "Double homeobox protein A",
  "gene_symbol": "DUXA"
}